{
  "term_id": "GO:0030316",
  "gene_name": "Macrophage colony-stimulating factor 1",
  "gene": "UniProtKB:P09603",
  "gene_symbol": "CSF1",
  "term_label": "osteoclast differentiation"
}